maintenance of transcriptional fidelity during transcription elongation by RNA polymerase II [GO:0001193] (BP) References: PMID:14531857, PMID:16492753, PMID:17535246 Sources: GOC:txnOH Definition: Suppression of the occurrence of transcriptional errors, such as substitutions and/or insertions of nucleotides that do not correctly match the template base, during the process of transcription elongation from an RNA polymerase II promoter. Also known as: maintenance of transcriptional fidelity during DNA-dependent transcription elongation from RNA polymerase II promoter, maintenance of transcriptional fidelity during DNA-templated transcription elongation from RNA polymerase II promoter Relationships: is a type of maintenance of transcriptional fidelity during transcription elongation [GO:0001192]; is part of transcription elongation by RNA polymerase II [GO:0006368]